{
  "gene": "UniProtKB:P09093",
  "term_id": "GO:0006508",
  "term_label": "proteolysis",
  "gene_symbol": "CELA3A",
  "gene_name": "Chymotrypsin-like elastase family member 3A"
}